response to cyclopentenone [GO:0010583] (biological process) Subtypes: cellular response to cyclopentenone [GO:0071410] Relationships: is a type of response to chemical [GO:0042221] Definition: Any process that results in a change in state or activity of a cell or an organism (in terms of movement, secretion, enzyme production, gene expression, etc.) as a result of a cyclopentenone stimulus. Cyclopentenones are oxylipins derived from polyunsaturated fatty acids. They are structurally similar to jasmonic acid, but contain a reactive unsaturated carbonyl structure in the cyclo-ring. Cyclopentenones include phytoprostanes and 12-oxo-phytodienoic acid. References: PMID:18334669